{
  "gene": "UniProtKB:P08842",
  "term_id": "UNKNOWN:0002",
  "gene_name": "Steryl-sulfatase",
  "term_label": "Unknown biological process",
  "gene_symbol": "STS"
}